positive regulation of apoptotic DNA fragmentation [GO:1902512] (biological process) References: PMID:15572351 Sources: GOC:TermGenie, GOC:hjd Definition: Any process that activates or increases the frequency, rate or extent of apoptotic DNA fragmentation. Relationships: is_a GO:1902510; is a type of positive regulation of DNA catabolic process [GO:1903626]; RO_0002213 apoptotic DNA fragmentation [GO:0006309] Also known as: positive regulation of DNA catabolic process during apoptosis, positive regulation of DNA catabolism during apoptosis, positive regulation of DNA fragmentation involved in apoptotic nuclear change, positive regulation of endonucleolytic DNA catabolic process involved in apoptosis, up regulation of DNA catabolic process during apoptosis, up regulation of DNA catabolism during apoptosis, up regulation of DNA fragmentation involved in apoptotic nuclear change, up regulation of apoptotic DNA fragmentation, up regulation of endonucleolytic DNA catabolic process involved in apoptosis, up-regulation of DNA catabolic process during apoptosis, up-regulation of DNA catabolism during apoptosis, up-regulation of DNA fragmentation involved in apoptotic nuclear change, up-regulation of apoptotic DNA fragmentation, up-regulation of endonucleolytic DNA catabolic process involved in apoptosis, upregulation of DNA catabolic process during apoptosis, upregulation of DNA catabolism during apoptosis, upregulation of DNA fragmentation involved in apoptotic nuclear change, upregulation of apoptotic DNA fragmentation, upregulation of endonucleolytic DNA catabolic process involved in apoptosis, activation of DNA catabolic process during apoptosis, activation of DNA catabolism during apoptosis, activation of DNA fragmentation involved in apoptotic nuclear change, activation of apoptotic DNA fragmentation, activation of endonucleolytic DNA catabolic process involved in apoptosis